forebrain astrocyte development [GO:0021897] (biological process) Definition: The process aimed at the progression of an astrocyte that resides in the forebrain, from initial commitment of the cell to its fate, to the fully functional differentiated cell. An astrocyte is the most abundant type of glial cell. Astrocytes provide support for neurons and regulate the environment in which they function. Sources: GOC:cls, GOC:dgh, GOC:dph, GOC:jid, GO_REF:0000021 Relationships: is a type of astrocyte development [GO:0014002]; is part of forebrain astrocyte differentiation [GO:0021896]